{
  "term_id": "GO:0043161",
  "gene": "UniProtKB:Q9UH77",
  "gene_symbol": "KLHL3",
  "term_label": "proteasome-mediated ubiquitin-dependent protein catabolic process",
  "gene_name": "Kelch-like protein 3"
}